intracellular acyl-CoA homeostasis [GO:0042049] (biological process) Relationships: is a type of intracellular chemical homeostasis [GO:0055082] Also known as: cell acyl-CoA homeostasis, cellular acyl-CoA homeostasis Definition: A homeostatic process involved in the maintenance of a steady state level of acyl-CoA within a cell. Sources: GOC:ai, GOC:dph, GOC:tb